{
  "gene": "UniProtKB:A0A0B4J2A2",
  "term_id": "GO:0003755",
  "gene_name": "Peptidyl-prolyl cis-trans isomerase A-like 4C",
  "gene_symbol": "PPIAL4C",
  "term_label": "peptidyl-prolyl cis-trans isomerase activity"
}